{
  "term_label": "Unknown molecular function",
  "term_id": "UNKNOWN:0001",
  "gene": "UniProtKB:Q8N8D9",
  "gene_symbol": "IRF1-AS1",
  "gene_name": "Uncharacterized protein IRF1-AS1"
}